{
  "gene": "UniProtKB:Q7Z4Y8",
  "term_id": "GO:0046933",
  "gene_name": "Putative ATP synthase subunit g 2, mitochondrial",
  "term_label": "proton-transporting ATP synthase activity, rotational mechanism",
  "gene_symbol": "ATP5MGL"
}